cellular response to capsazepine [GO:0072761] (biological process) Sources: GOC:mah Relationships: is a type of response to capsazepine [GO:1901594] Definition: Any process that results in a change in state or activity of a cell (in terms of movement, secretion, enzyme production, gene expression, etc.) as a result of a capsazepine stimulus.